{
  "gene": "UniProtKB:Q9UQN3",
  "gene_name": "Charged multivesicular body protein 2b",
  "gene_symbol": "CHMP2B",
  "term_id": "GO:0000815",
  "term_label": "ESCRT III complex"
}